{
  "gene_name": "TBC1 domain family member 3B",
  "term_id": "GO:0005096",
  "gene_symbol": "TBC1D3B",
  "gene": "UniProtKB:A6NDS4",
  "term_label": "GTPase activator activity"
}